positive regulation of oocyte development [GO:0060282] (biological process) Relationships: is a type of positive regulation of cell development [GO:0010720]; is a type of regulation of oocyte development [GO:0060281]; is a type of positive regulation of reproductive process [GO:2000243]; positively regulates oocyte development [GO:0048599] Sources: GOC:dph, GOC:tb Definition: Any process that increases the rate or extent of the process whose specific outcome is the progression of an oocyte over time, from initial commitment of the cell to its specific fate, to the fully functional differentiated cell.